negative regulation of cellular response to heat [GO:1900035] (biological process) Also known as: down regulation of cellular response to heat stress, down-regulation of cellular response to heat stress, downregulation of cellular response to heat stress, inhibition of cellular response to heat stress, negative regulation of cellular response to heat stress, down regulation of cellular response to heat, down-regulation of cellular response to heat, downregulation of cellular response to heat, inhibition of cellular response to heat Relationships: is a type of negative regulation of cellular process [GO:0048523]; is a type of negative regulation of response to stimulus [GO:0048585]; is a type of regulation of cellular response to heat [GO:1900034]; negatively regulates cellular response to heat [GO:0034605] Definition: Any process that stops, prevents or reduces the frequency, rate or extent of cellular response to heat. Sources: GOC:TermGenie, GOC:yaf